mycinamicin VI 2''-O-methyltransferase activity [GO:0102302] (molecular function) Definition: Catalysis of the reaction: S-adenosyl-L-methionine + mycinamicin VI = S-adenosyl-L-homocysteine + mycinamicin III(1+) + H+. Sources: EC:2.1.1.238, GOC:pz Relationships: is_a methyltransferase activity [GO:0008168]